{
  "term_id": "UNKNOWN:0002",
  "gene_name": "Testis development-related protein 1",
  "gene": "UniProtKB:Q3Y452",
  "term_label": "Unknown biological process",
  "gene_symbol": "TDRG1"
}